ISWI-type complex [GO:0031010] (CC) Definition: Any nuclear protein complex that contains an ATPase subunit of the imitation switch (ISWI) family. ISWI ATPases are involved in assembling chromatin and in sliding and spacing nucleosomes to regulate transcription of nuclear RNA polymerases I, II, and III and also DNA replication, recombination and repair. References: PMID:15020051, PMID:15284901, PMID:16568949, PMID:21810179 Sources: GOC:krc, GOC:mah Relationships: is a type of GO:0070603 Subtypes: CHRAC [GO:0008623], Isw1 complex [GO:0016587], NURF complex [GO:0016589], ACF complex [GO:0016590], GO:0031213, WICH complex [GO:0090535], NoRC complex [GO:0090536], GO:0090537